{
  "gene": "UniProtKB:P35749",
  "gene_name": "Myosin-11",
  "gene_symbol": "MYH11",
  "term_label": "myosin II complex",
  "term_id": "GO:0016460"
}